{
  "gene_name": "Alpha-1D adrenergic receptor",
  "term_id": "GO:0043410",
  "gene_symbol": "ADRA1D",
  "gene": "UniProtKB:P25100",
  "term_label": "positive regulation of MAPK cascade"
}